regulation of amniotic stem cell differentiation [GO:2000797] (biological process) Definition: Any process that modulates the frequency, rate or extent of amniotic stem cell differentiation. Sources: GOC:obol Relationships: is a type of regulation of mesenchymal stem cell differentiation [GO:2000739]; regulates amniotic stem cell differentiation [GO:0097086] Subtypes: negative regulation of amniotic stem cell differentiation [GO:2000798], positive regulation of amniotic stem cell differentiation [GO:2000799]